{
  "gene": "UniProtKB:B2RN74",
  "term_label": "Unknown cellular component",
  "gene_symbol": "OR11H12",
  "term_id": "UNKNOWN:0003",
  "gene_name": "Olfactory receptor 11H12"
}